{
  "gene_name": "Endoplasmic reticulum aminopeptidase 2",
  "gene_symbol": "ERAP2",
  "term_label": "proteolysis",
  "gene": "UniProtKB:Q6P179",
  "term_id": "GO:0006508"
}